{
  "term_id": "GO:0070383",
  "gene_symbol": "APOBEC3H",
  "term_label": "DNA cytosine deamination",
  "gene": "UniProtKB:Q6NTF7",
  "gene_name": "DNA dC-dU-editing enzyme APOBEC-3H"
}